negative regulation of phospholipid translocation [GO:0061093] (biological process) Definition: Any process that decreases the frequency, rate or extent of the translocation, or flipping, of phospholipid molecules from one monolayer of a membrane bilayer to the opposite monolayer. Subtypes: GO:1905781 Relationships: is a type of negative regulation of cellular component organization [GO:0051129]; is a type of GO:0061091; is a type of GO:2001139; negatively regulates phospholipid translocation [GO:0045332] References: PMID:19966303 Sources: GOC:dph, GOC:jh, GOC:tb